{
  "term_id": "GO:0005525",
  "term_label": "GTP binding",
  "gene_name": "Guanylate-binding protein 1",
  "gene_symbol": "GBP1",
  "gene": "UniProtKB:P32455"
}